{
  "gene": "UniProtKB:O00178",
  "term_label": "Unknown cellular component",
  "gene_symbol": "GTPBP1",
  "gene_name": "GTP-binding protein 1",
  "term_id": "UNKNOWN:0003"
}